{
  "gene_name": "Tubulin monoglutamylase TTLL4",
  "term_id": "GO:0070740",
  "term_label": "tubulin-glutamic acid ligase activity",
  "gene": "UniProtKB:Q14679",
  "gene_symbol": "TTLL4"
}